{
  "gene": "UniProtKB:Q8NGF1",
  "gene_symbol": "OR52R1",
  "term_label": "plasma membrane",
  "term_id": "GO:0005886",
  "gene_name": "Olfactory receptor 52R1"
}